{
  "term_label": "long-chain fatty acyl-CoA hydrolase activity",
  "term_id": "GO:0052816",
  "gene_symbol": "THEM5",
  "gene_name": "Acyl-coenzyme A thioesterase THEM5",
  "gene": "UniProtKB:Q8N1Q8"
}